{
  "gene": "UniProtKB:O43900",
  "gene_symbol": "PRICKLE3",
  "term_id": "UNKNOWN:0003",
  "term_label": "Unknown cellular component",
  "gene_name": "Prickle planar cell polarity protein 3"
}